{
  "term_label": "TAP1 binding",
  "gene_symbol": "TAP1",
  "gene": "UniProtKB:Q03518",
  "term_id": "GO:0046978",
  "gene_name": "Antigen peptide transporter 1"
}